{
  "gene_symbol": "PRKAB1",
  "term_label": "protein kinase binding",
  "gene": "UniProtKB:Q9Y478",
  "gene_name": "5'-AMP-activated protein kinase subunit beta-1",
  "term_id": "GO:0019901"
}